{
  "gene_name": "CTP synthase 2",
  "term_id": "GO:0005737",
  "gene_symbol": "CTPS2",
  "gene": "UniProtKB:Q9NRF8",
  "term_label": "cytoplasm"
}